{
  "term_label": "kinetochore",
  "gene_symbol": "BUB3",
  "gene": "UniProtKB:O43684",
  "term_id": "GO:0000776",
  "gene_name": "Mitotic checkpoint protein BUB3"
}